P-methyltransferase activity [GO:0051994] (molecular function) Definition: Catalysis of the transfer of a methyl group to the phosphorus atom of an acceptor molecule. Sources: GOC:ai Relationships: is a type of methyltransferase activity [GO:0008168]